{
  "gene_name": "Homeobox protein SIX4",
  "term_label": "RNA polymerase II cis-regulatory region sequence-specific DNA binding",
  "gene": "UniProtKB:Q9UIU6",
  "term_id": "GO:0000978",
  "gene_symbol": "SIX4"
}